{
  "gene_symbol": "CENPV",
  "gene_name": "Centromere protein V",
  "gene": "UniProtKB:Q7Z7K6",
  "term_label": "pericentric heterochromatin formation",
  "term_id": "GO:0031508"
}